{
  "term_label": "RNA polymerase II cis-regulatory region sequence-specific DNA binding",
  "gene_name": "Paired box protein Pax-4",
  "gene": "UniProtKB:O43316",
  "term_id": "GO:0000978",
  "gene_symbol": "PAX4"
}